{
  "gene": "UniProtKB:Q9NPI6",
  "term_label": "deadenylation-independent decapping of nuclear-transcribed mRNA",
  "term_id": "GO:0031087",
  "gene_symbol": "DCP1A",
  "gene_name": "mRNA-decapping enzyme 1A"
}